{
  "term_label": "DNA-binding transcription activator activity, RNA polymerase II-specific",
  "gene_name": "Transcription factor AP-2 gamma",
  "term_id": "GO:0001228",
  "gene": "UniProtKB:Q92754",
  "gene_symbol": "TFAP2C"
}